{
  "term_id": "GO:0003700",
  "term_label": "DNA-binding transcription factor activity",
  "gene_symbol": "PRDM5",
  "gene": "UniProtKB:Q9NQX1",
  "gene_name": "PR domain zinc finger protein 5"
}